{
  "gene": "UniProtKB:Q9ULE4",
  "gene_symbol": "FAM184B",
  "gene_name": "Protein FAM184B",
  "term_label": "Unknown biological process",
  "term_id": "UNKNOWN:0002"
}